positive regulation of cell growth [GO:0030307] (BP) Also known as: up regulation of cell growth, up-regulation of cell growth, upregulation of cell growth, activation of cell growth, stimulation of cell growth Sources: GOC:go_curators Subtypes: GO:0045773, GO:0048672, positive regulation of sprouting of injured axon [GO:0048687], positive regulation of unidimensional cell growth [GO:0051512], GO:0061051, positive regulation of direction of cell growth [GO:0061390], GO:1902892, positive regulation of chondrocyte hypertrophy [GO:1903043], positive regulation of dendrite extension [GO:1903861], positive regulation of pseudohyphal growth [GO:2000222] Relationships: is a type of regulation of cell growth [GO:0001558]; is a type of positive regulation of growth [GO:0045927]; is a type of positive regulation of cellular process [GO:0048522]; positively regulates cell growth [GO:0016049] Definition: Any process that activates or increases the frequency, rate, extent or direction of cell growth.